{
  "gene_name": "Sodium-dependent serotonin transporter",
  "term_label": "neuron projection",
  "gene_symbol": "SLC6A4",
  "gene": "UniProtKB:P31645",
  "term_id": "GO:0043005"
}